{
  "gene": "UniProtKB:Q6ZMG9",
  "gene_name": "Ceramide synthase 6",
  "term_id": "GO:0050291",
  "gene_symbol": "CERS6",
  "term_label": "sphingosine N-acyltransferase activity"
}